galactose-1-phosphate thymidylyltransferase activity [GO:0047342] (molecular function) Relationships: is a type of nucleotidyltransferase activity [GO:0016779] Sources: EC:2.7.7.32, RHEA:17165 Definition: Catalysis of the reaction: alpha-D-galactose 1-phosphate + dTTP = diphosphate + dTDP-D-galactose. Also known as: dTDP galactose pyrophosphorylase activity, dTDP-galactose diphosphorylase activity, dTDP-galactose pyrophosphorylase activity, dTTP:alpha-D-galactose-1-phosphate thymidylyltransferase activity, galactose 1-phosphate thymidylyl transferase activity, thymidine diphosphogalactose pyrophosphorylase activity, thymidine triphosphate:alpha-D-galactose 1-phosphate thymidylyltransferase activity